cocaine binding [GO:0019811] (molecular function) Relationships: is_a cation binding [GO:0043169]; is a type of heterocyclic compound binding [GO:1901363] Definition: Binding to cocaine (2-beta-carbomethoxy-3-beta-benzoxytropane), an alkaloid obtained from dried leaves of the South American shrub Erythroxylon coca or by chemical synthesis. Sources: GOC:jl, ISBN:0198506732